{
  "term_id": "GO:0046933",
  "gene_symbol": "ATP5MF",
  "gene_name": "ATP synthase subunit f, mitochondrial",
  "gene": "UniProtKB:P56134",
  "term_label": "proton-transporting ATP synthase activity, rotational mechanism"
}